{
  "gene_name": "Cysteine--tRNA ligase, cytoplasmic",
  "gene_symbol": "CARS1",
  "term_label": "cytoplasm",
  "gene": "UniProtKB:P49589",
  "term_id": "GO:0005737"
}